{
  "gene_name": "Transmembrane protein 182",
  "term_id": "UNKNOWN:0001",
  "gene_symbol": "TMEM182",
  "gene": "UniProtKB:Q6ZP80",
  "term_label": "Unknown molecular function"
}